{
  "gene_symbol": "SRD5A2",
  "term_label": "male gonad development",
  "gene": "UniProtKB:P31213",
  "term_id": "GO:0008584",
  "gene_name": "3-oxo-5-alpha-steroid 4-dehydrogenase 2"
}